{
  "gene_name": "Olfactory receptor 51T1",
  "term_id": "UNKNOWN:0002",
  "gene": "UniProtKB:Q8NGJ9",
  "gene_symbol": "OR51T1",
  "term_label": "Unknown biological process"
}